transferase complex, transferring phosphorus-containing groups [GO:0061695] (cellular component) Sources: GOC:bhm, GOC:dph Definition: A transferase complex capable of catalysis of the transfer of a phosphorus-containing group from one compound (donor) to another (acceptor). Subtypes: telomerase catalytic core complex [GO:0000333], creatine kinase complex [GO:0002185], ribose phosphate diphosphokinase complex [GO:0002189], phosphatidylinositol 3-kinase complex [GO:0005942], 6-phosphofructokinase complex [GO:0005945], protein-N(PI)-phosphohistidine-sugar phosphotransferase complex [GO:0009357], GO:0009358, RNA polymerase complex [GO:0030880], DNA polymerase complex [GO:0042575], 6-phosphofructo-2-kinase/fructose-2,6-biphosphatase complex [GO:0043540], UDP-N-acetylglucosamine transferase complex [GO:0043541], alpha-D-ribose 1-methylphosphonate 5-triphosphate synthase complex [GO:0061694], UDP-N-acetylglucosamine-lysosomal-enzyme N-acetylglucosaminephosphotransferase complex [GO:0070622], PAS complex [GO:0070772], GO:0106098, GDP-mannose pyrophosphorylase complex [GO:0120508], adenylyltransferase complex [GO:1902503], protein kinase complex [GO:1902911], GO:1902912 Relationships: is a type of transferase complex [GO:1990234]